{
  "term_label": "translational initiation",
  "gene_name": "Eukaryotic translation initiation factor 3 subunit H",
  "gene": "UniProtKB:O15372",
  "term_id": "GO:0006413",
  "gene_symbol": "EIF3H"
}